{
  "term_label": "cell-cell junction",
  "gene": "UniProtKB:P17661",
  "term_id": "GO:0005911",
  "gene_name": "Desmin",
  "gene_symbol": "DES"
}